flavanone 7-O-beta-glucosyltransferase activity [GO:0047243] (molecular function) Relationships: is a type of GO:0035251 Sources: EC:2.4.1.185, MetaCyc:2.4.1.185-RXN Definition: Catalysis of the reaction: a flavanone + UDP-D-glucose = a flavanone 7-O-beta-D-glucoside + UDP. Also known as: UDP-glucose:flavanone 7-O-beta-D-glucosyltransferase activity, UDPglucose:flavanone 7-O-beta-D-glucosyltransferase activity, hesperetin 7-O-glucosyl-transferase activity, naringenin 7-O-glucosyltransferase activity, uridine diphosphoglucose-flavanone 7-O-glucosyltransferase activity